{
  "gene_symbol": "SHISAL2B",
  "term_id": "UNKNOWN:0002",
  "gene_name": "Protein shisa-like-2B",
  "term_label": "Unknown biological process",
  "gene": "UniProtKB:A6NKW6"
}